{
  "gene": "UniProtKB:O75396",
  "term_label": "Unknown biological process",
  "term_id": "UNKNOWN:0002",
  "gene_symbol": "SEC22B",
  "gene_name": "Vesicle-trafficking protein SEC22b"
}